{
  "gene_symbol": "SMARCA1",
  "gene_name": "Probable global transcription activator SNF2L1",
  "term_label": "chromatin binding",
  "term_id": "GO:0003682",
  "gene": "UniProtKB:P28370"
}